radial glial cell differentiation [GO:0060019] (biological process) Relationships: is a type of glial cell differentiation [GO:0010001] Subtypes: spinal cord radial glial cell differentiation [GO:0021531], forebrain radial glial cell differentiation [GO:0021861] Definition: The process in which neuroepithelial cells of the neural tube give rise to radial glial cells, specialized bipotential progenitors cells of the brain. Differentiation includes the processes involved in commitment of a cell to a specific fate. Sources: GOC:dph